{
  "gene_symbol": "CEBPZOS",
  "gene_name": "Protein CEBPZOS",
  "term_label": "Unknown cellular component",
  "term_id": "UNKNOWN:0003",
  "gene": "UniProtKB:A8MTT3"
}